{
  "gene_symbol": "MEIS3",
  "gene_name": "Homeobox protein Meis3",
  "gene": "UniProtKB:Q99687",
  "term_id": "GO:0000978",
  "term_label": "RNA polymerase II cis-regulatory region sequence-specific DNA binding"
}